pentitol metabolic process [GO:0019519] (biological process) Relationships: is a type of GO:0005975; is_a GO:0019751 Subtypes: pentitol biosynthetic process [GO:0019526], pentitol catabolic process [GO:0019527], xylitol metabolic process [GO:0051164] Sources: ISBN:0198506732 Definition: The chemical reactions and pathways involving pentitols, any alditol with a chain of five carbon atoms in the molecule. Also known as: pentitol metabolism